{
  "gene_symbol": "CDC7",
  "term_label": "protein serine/threonine kinase activity",
  "gene": "UniProtKB:O00311",
  "gene_name": "Cell division cycle 7-related protein kinase",
  "term_id": "GO:0004674"
}